{
  "gene": "UniProtKB:Q8N292",
  "gene_symbol": "GAPT",
  "gene_name": "Protein GAPT",
  "term_id": "GO:0005886",
  "term_label": "plasma membrane"
}